{
  "term_label": "fatty-acyl-CoA biosynthetic process",
  "gene_name": "Glutaryl-CoA dehydrogenase, mitochondrial",
  "gene_symbol": "GCDH",
  "gene": "UniProtKB:Q92947",
  "term_id": "GO:0046949"
}